{
  "gene_symbol": "IL36G",
  "gene_name": "Interleukin-36 gamma",
  "gene": "UniProtKB:Q9NZH8",
  "term_label": "cytokine activity",
  "term_id": "GO:0005125"
}